{
  "gene_symbol": "OR5K2",
  "gene_name": "Olfactory receptor 5K2",
  "term_label": "Unknown biological process",
  "gene": "UniProtKB:Q8NHB8",
  "term_id": "UNKNOWN:0002"
}